{
  "gene_symbol": "FAM72D",
  "gene_name": "Protein FAM72D",
  "gene": "UniProtKB:Q6L9T8",
  "term_id": "UNKNOWN:0002",
  "term_label": "Unknown biological process"
}